DNA translocase activity [GO:0015616] (molecular function) Definition: Generation of movement along a single- or double-stranded DNA molecule, driven by ATP hydrolysis. References: PMID:16428451, PMID:17631491 Sources: GOC:mah Note: Note that some gene products that possess DNA translocase activity, such as members of the FtsK/SpoIIIE family, can be fixed in place by interactions with other components of the cell; the relative movement between the protein and DNA bound to it results in movement of the DNA within the cell, often across a membrane. Relationships: is a type of GO:0008094; has part DNA binding [GO:0003677] Subtypes: type I site-specific deoxyribonuclease activity [GO:0009035], GO:0140584